{
  "term_label": "cytoplasm",
  "term_id": "GO:0005737",
  "gene_symbol": "CLIC3",
  "gene_name": "Chloride intracellular channel protein 3",
  "gene": "UniProtKB:O95833"
}